{
  "gene_name": "Melanoma-associated antigen C3",
  "gene": "UniProtKB:Q8TD91",
  "gene_symbol": "MAGEC3",
  "term_id": "UNKNOWN:0001",
  "term_label": "Unknown molecular function"
}